{
  "gene_name": "Prorelaxin H2",
  "term_label": "Unknown cellular component",
  "gene": "UniProtKB:P04090",
  "gene_symbol": "RLN2",
  "term_id": "UNKNOWN:0003"
}